{
  "gene": "UniProtKB:Q13409",
  "gene_symbol": "DYNC1I2",
  "gene_name": "Cytoplasmic dynein 1 intermediate chain 2",
  "term_label": "dynein heavy chain binding",
  "term_id": "GO:0045504"
}